nucleoside kinase activity [GO:0019206] (MF) Definition: Catalysis of the reaction: ATP + nucleoside = ADP + nucleoside monophosphate. Sources: GOC:ai Subtypes: adenosine kinase activity [GO:0004001], uridine kinase activity [GO:0004849], cytidine kinase activity [GO:0043771], guanosine kinase activity [GO:0106366] Relationships: is_a GO:0016773; is a type of nucleobase-containing compound kinase activity [GO:0019205]; is part of nucleotide biosynthetic process [GO:0009165]